prostaglandin metabolic process [GO:0006693] (biological process) Definition: The chemical reactions and pathways involving prostaglandins, any of a group of biologically active metabolites which contain a cyclopentane ring due to the formation of a bond between two carbons of a fatty acid. They have a wide range of biological activities. Sources: ISBN:0198506732 Also known as: prostaglandin metabolism Relationships: is a type of prostanoid metabolic process [GO:0006692] Subtypes: prostaglandin biosynthetic process [GO:0001516]